calcium ion transmembrane transporter activity [GO:0015085] (molecular function) Relationships: is a type of GO:0046873; is part of GO:0070588 Subtypes: calcium channel activity [GO:0005262], P-type calcium transporter activity [GO:0005388], calcium:monoatomic cation antiporter activity [GO:0015368] Definition: Enables the transfer of calcium (Ca) ions from one side of a membrane to the other. Regulation: negatively regulated by negative regulation of calcium ion transmembrane transporter activity [GO:1901020] Sources: GOC:dgf